{
  "term_label": "ribosome biogenesis",
  "term_id": "GO:0042254",
  "gene_name": "Ribosomal biogenesis factor",
  "gene": "UniProtKB:Q8N0T1",
  "gene_symbol": "RBIS"
}